{
  "gene_symbol": "PHETA2",
  "gene_name": "Sesquipedalian-2",
  "term_label": "Unknown molecular function",
  "gene": "UniProtKB:Q6ICB4",
  "term_id": "UNKNOWN:0001"
}